{
  "gene_symbol": "MTOR",
  "term_id": "GO:0016242",
  "gene_name": "Serine_threonine-protein kinase mTOR",
  "gene": "UniProtKB:P42345",
  "term_label": "negative regulation of macroautophagy"
}